negative regulation of adenylate cyclase-activating adrenergic receptor signaling pathway involved in heart process [GO:0140199] (biological process) Definition: Any process that stops, prevents or reduces the frequency, rate or extent of an adenylate cyclase-activating adrenergic receptor signaling pathway involved in some heart process. Sources: GOC:BHF, GOC:BHF_miRNA, GOC:rph Relationships: is a type of negative regulation of multicellular organismal process [GO:0051241]; is a type of GO:0071878; negatively regulates GO:0086023